{
  "gene_name": "Microtubule-associated protein 1B",
  "gene_symbol": "MAP1B",
  "gene": "UniProtKB:P46821",
  "term_label": "dendrite",
  "term_id": "GO:0030425"
}